motogenic signaling initiating cell movement in cerebral cortex [GO:0021807] (BP) Subtypes: growth factor signaling initiating cell movement involved in cerebral cortex radial glia guided migration [GO:0021811] Relationships: is a type of cell communication [GO:0007154]; is a type of GO:0023052; is part of initiation of movement involved in cerebral cortex radial glia guided migration [GO:0021806] References: PMID:12626695 Sources: GOC:cls, GOC:dgh, GOC:dph, GOC:jid, GO_REF:0000021 Also known as: motogenic signalling initiating cell movement in the cerebral cortex Definition: The interaction of soluble factors and receptors that result in the movement of cells in the primitive cerebral cortex.